{
  "gene": "UniProtKB:Q9HD87",
  "term_label": "Unknown biological process",
  "gene_symbol": "C6orf50",
  "term_id": "UNKNOWN:0002",
  "gene_name": "Putative uncharacterized protein C6orf50"
}